{
  "gene_symbol": "Q96M85",
  "term_id": "UNKNOWN:0002",
  "gene_name": "Putative uncharacterized protein FLJ32756",
  "gene": "UniProtKB:Q96M85",
  "term_label": "Unknown biological process"
}